leading edge membrane [GO:0031256] (cellular component) Definition: The portion of the plasma membrane surrounding the leading edge of a motile cell. Relationships: is a type of GO:0110165; is part of GO:0005886; BFO_0000050 GO:0031252 Subtypes: lamellipodium membrane [GO:0031258], ruffle membrane [GO:0032587], GO:0032589 Sources: GOC:mah